positive regulation of protein acetylation [GO:1901985] (biological process) Also known as: positive regulation of protein amino acid acetylation, up regulation of protein acetylation, up regulation of protein amino acid acetylation, up-regulation of protein acetylation, up-regulation of protein amino acid acetylation, upregulation of protein acetylation, upregulation of protein amino acid acetylation, activation of protein acetylation, activation of protein amino acid acetylation References: PMID:22117195 Sources: GOC:TermGenie Subtypes: positive regulation of N-terminal peptidyl-methionine acetylation [GO:1904665], GO:2000758 Relationships: is a type of positive regulation of protein modification process [GO:0031401]; is a type of regulation of protein acetylation [GO:1901983]; positively regulates GO:0006473 Definition: Any process that activates or increases the frequency, rate or extent of protein acetylation.